{
  "gene_name": "Angiopoietin-related protein 3",
  "term_label": "extracellular matrix",
  "gene": "UniProtKB:Q9Y5C1",
  "gene_symbol": "ANGPTL3",
  "term_id": "GO:0031012"
}